{
  "gene_symbol": "C2orf16",
  "gene_name": "Uncharacterized protein C2orf16",
  "gene": "UniProtKB:Q68DN1",
  "term_label": "Unknown biological process",
  "term_id": "UNKNOWN:0002"
}